{
  "gene_symbol": "PRKCB",
  "term_label": "intracellular signal transduction",
  "gene_name": "Protein kinase C beta type",
  "gene": "UniProtKB:P05771",
  "term_id": "GO:0035556"
}